{
  "term_id": "GO:0007605",
  "gene": "UniProtKB:Q8WXR4",
  "gene_symbol": "MYO3B",
  "term_label": "sensory perception of sound",
  "gene_name": "Myosin-IIIb"
}